{
  "term_id": "GO:0003823",
  "term_label": "antigen binding",
  "gene_name": "Immunoglobulin heavy variable 4-34",
  "gene_symbol": "IGHV4-34",
  "gene": "UniProtKB:P06331"
}